{
  "term_label": "regulation of transcription by RNA polymerase II",
  "gene": "UniProtKB:Q7LBC6",
  "gene_symbol": "KDM3B",
  "gene_name": "Lysine-specific demethylase 3B",
  "term_id": "GO:0006357"
}